{
  "gene_symbol": "HLF",
  "term_id": "GO:0005634",
  "term_label": "nucleus",
  "gene": "UniProtKB:Q16534",
  "gene_name": "Hepatic leukemia factor"
}